{
  "gene": "UniProtKB:P19484",
  "term_id": "GO:0000981",
  "gene_name": "Transcription factor EB",
  "term_label": "DNA-binding transcription factor activity, RNA polymerase II-specific",
  "gene_symbol": "TFEB"
}